toluene oxidation to catechol [GO:0019604] (biological process) Definition: The formation from toluene of catechol, dihydroxybenzene, by successive oxidations followed by loss of carbon dioxide (CO2). Sources: MetaCyc:TOLUENE-DEG-CATECHOL-PWY Relationships: is a type of catechol-containing compound metabolic process [GO:0009712]; is a type of toluene oxidation [GO:0019600]